symbiont-mediated cAMP intoxication of host cell [GO:0141042] (biological process) Also known as: cAMP intoxication in host Relationships: is a type of symbiont-mediated perturbation of host signal transduction pathway [GO:0052027] References: PMID:16390441, PMID:19516256, PMID:27731909, PMID:33013916 Definition: The production by a symbiont of high levels of cyclic AMP in a host cell, impairing host cellular functions in multiple ways, including ATP depletion, interference with host intracellular signaling, cytoskeletal defects and apoptosis-related cell death. The host is defined as the larger of the organisms involved in a symbiotic interaction.